{
  "gene_symbol": "SAMSN1",
  "term_id": "GO:0050869",
  "gene_name": "SAM domain-containing protein SAMSN-1",
  "term_label": "negative regulation of B cell activation",
  "gene": "UniProtKB:Q9NSI8"
}